{
  "gene": "UniProtKB:P0C6A0",
  "term_label": "spermatogenesis",
  "gene_symbol": "ZGLP1",
  "term_id": "GO:0007283",
  "gene_name": "GATA-type zinc finger protein 1"
}